{
  "term_label": "morphogenesis of an epithelium",
  "gene_symbol": "KRT37",
  "term_id": "GO:0002009",
  "gene_name": "Keratin, type I cuticular Ha7",
  "gene": "UniProtKB:O76014"
}